{
  "term_id": "UNKNOWN:0001",
  "gene_name": "Solute carrier family 66 member 3",
  "term_label": "Unknown molecular function",
  "gene": "UniProtKB:Q8N755",
  "gene_symbol": "SLC66A3"
}